orexin receptor binding [GO:0042324] (molecular function) Also known as: hypocretin receptor binding, hypocretin receptor ligand, orexin receptor ligand Relationships: is a type of neuropeptide receptor binding [GO:0071855] Definition: Binding to an orexin receptor. References: PMID:11988773 Sources: GOC:ceb Subtypes: type 1 orexin receptor binding [GO:0031771], type 2 orexin receptor binding [GO:0031772]